{
  "gene_symbol": "ZDHHC3",
  "term_label": "protein-cysteine S-palmitoyltransferase activity",
  "term_id": "GO:0019706",
  "gene": "UniProtKB:Q9NYG2",
  "gene_name": "Palmitoyltransferase ZDHHC3"
}